deoxynucleoside kinase activity [GO:0019136] (molecular function) Definition: Catalysis of the reaction: ATP + 2'-deoxynucleoside = ADP + 2'-deoxynucleoside 5'-phosphate. Relationships: is_a nucleobase-containing compound kinase activity [GO:0019205]; is part of GO:0009157 Also known as: ATP:deoxynucleoside 5'-phosphotransferase activity, D. melanogaster deoxynucleoside kinase activity, Dm-dNK, Ms-dNK activity, ms-dNK, multifunctional deoxynucleoside kinase activity, multispecific deoxynucleoside kinase activity, multisubstrate deoxyribonucleoside kinase activity Sources: EC:2.7.1.145 Subtypes: deoxyadenosine kinase activity [GO:0004136], deoxycytidine kinase activity [GO:0004137], deoxyguanosine kinase activity [GO:0004138], thymidine kinase activity [GO:0004797]